{
  "gene": "UniProtKB:Q96PH1",
  "gene_symbol": "NOX5",
  "term_label": "superoxide anion generation",
  "gene_name": "NADPH oxidase 5",
  "term_id": "GO:0042554"
}